{
  "gene_name": "Protein CIST1",
  "term_label": "Unknown biological process",
  "gene": "UniProtKB:A0A2R8Y7Y5",
  "term_id": "UNKNOWN:0002",
  "gene_symbol": "CIST1"
}